GDP-2,4-diacetamido-2,4,6-trideoxy-alpha-D-glucopyranose hydrolase/2-epimerase activity [GO:0102224] (molecular function) Definition: Catalysis of the reaction: GDP-N,N'-diacetylbacillosamine + H2O = 2,4-diacetamido-2,4,6-trideoxy-alpha-D-mannopyranose + GDP + H+. Sources: RHEA:46316 Relationships: is a type of hydrolase activity, hydrolyzing O-glycosyl compounds [GO:0004553]